GTP cyclohydrolase IV activity [GO:0044682] (molecular function) Definition: Catalysis of the reaction: GTP + H2O = 7,8-dihydroneopterin 2',3'-cyclic phosphate + diphosphate + formate + H+. This activity is part of the biosynthesis of methanopterin in Archaea, and requires Fe2+. Also known as: Fe(2+)-dependent archaeal-specific GTP cyclohydrolase activity, archaeal-specific GTP cyclohydrolase activity, MptA activity Relationships: is a type of GTP cyclohydrolase activity [GO:0003933] References: PMID:17497938 Sources: GOC:mengo_curators, RHEA:25860